{
  "gene_name": "Germinal center-associated signaling and motility-like protein",
  "term_id": "UNKNOWN:0002",
  "gene": "UniProtKB:Q5JQS6",
  "gene_symbol": "GCSAML",
  "term_label": "Unknown biological process"
}